negative regulation of BMP signaling pathway [GO:0030514] (BP) Also known as: down regulation of BMP signaling pathway, down-regulation of BMP signaling pathway, downregulation of BMP signaling pathway, negative regulation of BMP signalling pathway, negative regulation of bone morphogenetic protein signaling pathway, negative regulation of bone morphogenetic protein signalling pathway, inhibition of BMP signaling pathway, negative regulation of decapentaplegic receptor signaling pathway, negative regulation of decapentaplegic receptor signalling pathway, negative regulation of decapentaplegic signaling pathway, negative regulation of BMP receptor signaling pathway Sources: GOC:go_curators Definition: Any process that stops, prevents, or reduces the frequency, rate or extent of the BMP signaling pathway. Relationships: is a type of regulation of BMP signaling pathway [GO:0030510]; is a type of negative regulation of transmembrane receptor protein serine/threonine kinase signaling pathway [GO:0090101]; is_a negative regulation of cellular response to growth factor stimulus [GO:0090288]; negatively regulates BMP signaling pathway [GO:0030509] Subtypes: sequestering of BMP in extracellular matrix [GO:0035582], sequestering of BMP from receptor via BMP binding [GO:0038098]